positive regulation of mammary stem cell proliferation [GO:2000103] (biological process) Relationships: is a type of positive regulation of cell population proliferation [GO:0008284]; is a type of positive regulation of developmental process [GO:0051094]; is a type of positive regulation of multicellular organismal process [GO:0051240]; is a type of regulation of mammary stem cell proliferation [GO:2000101]; positively regulates mammary stem cell proliferation [GO:0002174] Sources: GOC:obol Definition: Any process that activates or increases the frequency, rate or extent of mammary stem cell proliferation.